sphinganine-1-phosphate biosynthetic process [GO:0006669] (biological process) Relationships: is a type of sphinganine-1-phosphate metabolic process [GO:0006668]; is a type of phospholipid biosynthetic process [GO:0008654]; is a type of GO:0030148 Sources: GOC:ai Definition: The chemical reactions and pathways resulting in the formation of sphinganine-1-phosphate, the phosphorylated derivative of D-erythro-2-amino-1,3-octadecanediol. Also known as: dihydrosphingosine-1-phosphate biosynthesis, dihydrosphingosine-1-phosphate biosynthetic process, sphinganine-1-phosphate anabolism, sphinganine-1-phosphate biosynthesis, sphinganine-1-phosphate formation, sphinganine-1-phosphate synthesis